{
  "term_id": "GO:0001786",
  "gene": "UniProtKB:P13928",
  "gene_name": "Annexin A8",
  "term_label": "phosphatidylserine binding",
  "gene_symbol": "ANXA8"
}